{
  "gene_symbol": "RNF128",
  "gene_name": "E3 ubiquitin-protein ligase RNF128",
  "term_id": "GO:0005737",
  "term_label": "cytoplasm",
  "gene": "UniProtKB:Q8TEB7"
}